levopimaradiene synthase activity [GO:0052678] (molecular function) Definition: Catalysis of the reaction: (+)-copalyl diphosphate = abieta-8(14),12-diene + diphosphate. Also known as: ent-copalyl-diphosphate diphosphate-lyase [ent-abieta-8(14),12-diene-forming] activity Sources: RHEA:25548 Relationships: is a type of carbon-oxygen lyase activity, acting on phosphates [GO:0016838]